{
  "term_label": "Unknown molecular function",
  "gene_symbol": "ANKRD10",
  "term_id": "UNKNOWN:0001",
  "gene_name": "Ankyrin repeat domain-containing protein 10",
  "gene": "UniProtKB:Q9NXR5"
}